protein-carbohydrate complex subunit organization [GO:0071823] (biological process) Relationships: is a type of protein-containing complex organization [GO:0043933] Also known as: protein-carbohydrate complex subunit organisation Sources: GOC:mah Definition: Any process in which macromolecules aggregate, disaggregate, or are modified, resulting in the formation, disassembly, or alteration of a protein-carbohydrate complex. Subtypes: GO:0032985